oxygen sensor activity [GO:0019826] (molecular function) Sources: GOC:mah Definition: Binding to and responding, e.g. by conformational change, to changes in the cellular level of oxygen (O2). Relationships: is a type of GO:0140299; has part oxygen binding [GO:0019825]